{
  "gene_name": "Olfactory receptor 13A1",
  "gene_symbol": "OR13A1",
  "gene": "UniProtKB:Q8NGR1",
  "term_label": "Unknown cellular component",
  "term_id": "UNKNOWN:0003"
}